{
  "term_id": "GO:0005739",
  "term_label": "mitochondrion",
  "gene": "UniProtKB:Q9H061",
  "gene_symbol": "TMEM126A",
  "gene_name": "Transmembrane protein 126A"
}